{
  "gene": "UniProtKB:P35321",
  "term_label": "Unknown biological process",
  "gene_name": "Cornifin-A",
  "term_id": "UNKNOWN:0002",
  "gene_symbol": "SPRR1A"
}